{
  "gene": "UniProtKB:Q9HCK5",
  "gene_symbol": "AGO4",
  "gene_name": "Protein argonaute-4",
  "term_label": "RNA endonuclease activity",
  "term_id": "GO:0004521"
}